{
  "gene_symbol": "CYP7A1",
  "term_label": "cholesterol 7-alpha-monooxygenase activity",
  "gene_name": "Cytochrome P450 7A1",
  "term_id": "GO:0008123",
  "gene": "UniProtKB:P22680"
}